{
  "term_label": "signaling receptor binding",
  "gene_name": "Peripheral plasma membrane protein CASK",
  "gene_symbol": "CASK",
  "term_id": "GO:0005102",
  "gene": "UniProtKB:O14936"
}